gene silencing by siRNA-directed DNA methylation [GO:0080188] (BP) Subtypes: transposable element silencing by siRNA-mediated DNA methylation [GO:0141010] Definition: A small RNA-based gene silencing process in which small interfering RNAs (siRNAs) guide DNA methylation to the siRNA-generating genomic loci and other loci that are homologous to the siRNAs for de novo DNA methylation. This results in a heterochromatin assembly, a chromatin conformation that is refractory to transcription. In general this process consists of three phases: biogenesis of siRNAs, scaffold RNA production, and the formation of the guiding complex that recruits de novo DNA methyltransferases to the target loci. Transposable elements are silenced by this mechanism. Also known as: RdDM, RNA-directed DNA methylation, gene silencing by RNA-directed DNA methylation Relationships: is_a GO:0006346; is a type of siRNA-mediated heterochromatin formation [GO:0141194] References: PMID:21420348, PMID:33031395 Note: This process has been shown in plants and in yeasts, but so far has not been detected in vertebrates, organisms that lack RNA-dependent RNA polymerase.